{
  "gene": "UniProtKB:Q9H160",
  "gene_name": "Inhibitor of growth protein 2",
  "gene_symbol": "ING2",
  "term_id": "GO:0005634",
  "term_label": "nucleus"
}